{
  "term_label": "Unknown cellular component",
  "gene_symbol": "ATF7",
  "gene_name": "Cyclic AMP-dependent transcription factor ATF-7",
  "gene": "UniProtKB:P17544",
  "term_id": "UNKNOWN:0003"
}